{
  "term_label": "membrane",
  "term_id": "GO:0016020",
  "gene_symbol": "TAS2R46",
  "gene": "UniProtKB:P59540",
  "gene_name": "Taste receptor type 2 member 46"
}